{
  "gene": "UniProtKB:O43805",
  "gene_name": "Microtubule nucleation factor SSNA1",
  "term_label": "axon",
  "gene_symbol": "SSNA1",
  "term_id": "GO:0030424"
}